{
  "term_id": "GO:0045202",
  "gene_name": "Cytoplasmic polyadenylation element-binding protein 1",
  "gene_symbol": "CPEB1",
  "term_label": "synapse",
  "gene": "UniProtKB:Q9BZB8"
}